{
  "term_label": "D-glucose import",
  "term_id": "GO:0046323",
  "gene_name": "Solute carrier family 2, facilitated glucose transporter member 3",
  "gene_symbol": "SLC2A3",
  "gene": "UniProtKB:P11169"
}